{
  "gene": "UniProtKB:P98169",
  "term_label": "transcription coregulator activity",
  "gene_symbol": "ZXDB",
  "gene_name": "Zinc finger X-linked protein ZXDB",
  "term_id": "GO:0003712"
}